UMP salvage [GO:0044206] (BP) References: PMID:15096496 Sources: GOC:ecd Relationships: is a type of UMP biosynthetic process [GO:0006222]; is a type of GO:0010138 Definition: Any process which produces UMP, uridine monophosphate, from derivatives of it (e.g. cytidine, uridine, cytosine) without de novo synthesis. Also known as: UMP biosynthesis via nucleoside salvage pathway, UMP biosynthetic process via nucleoside salvage pathway